3-deoxy-2-octulosonidase activity [GO:0033937] (molecular function) Also known as: 2-keto-3-deoxyoctonate hydrolase activity, capsular-polysaccharide 3-deoxy-D-manno-2-octulosonohydrolase activity, octulofuranosylono hydrolase activity, octulopyranosylonohydrolase activity, octulosylono hydrolase activity Sources: EC:3.2.1.124 Relationships: is a type of hydrolase activity, hydrolyzing O-glycosyl compounds [GO:0004553] Definition: Catalysis of the endohydrolysis of the beta-ketopyranosidic linkages of 3-deoxy-D-manno-2-octulosonate in capsular polysaccharides.